{
  "gene_name": "Acyl-coenzyme A oxidase-like protein",
  "term_id": "GO:0033540",
  "term_label": "fatty acid beta-oxidation using acyl-CoA oxidase",
  "gene": "UniProtKB:Q9NUZ1",
  "gene_symbol": "ACOXL"
}